{
  "term_label": "Unknown molecular function",
  "gene_symbol": "Q6Q795",
  "term_id": "UNKNOWN:0001",
  "gene": "UniProtKB:Q6Q795",
  "gene_name": "Putative viral protein-binding protein C1"
}